{
  "term_label": "Unknown cellular component",
  "term_id": "UNKNOWN:0003",
  "gene_symbol": "PLEKHS1",
  "gene": "UniProtKB:Q5SXH7",
  "gene_name": "Pleckstrin homology domain-containing family S member 1"
}